pyrimidine deoxyribonucleoside catabolic process [GO:0046127] (biological process) Relationships: is a type of deoxyribonucleoside catabolic process [GO:0046121]; is a type of pyrimidine deoxyribonucleoside metabolic process [GO:0046125]; is a type of pyrimidine nucleoside catabolic process [GO:0046135] Also known as: pyrimidine deoxyribonucleoside breakdown, pyrimidine deoxyribonucleoside catabolism, pyrimidine deoxyribonucleoside degradation Subtypes: thymidine catabolic process [GO:0006214], GO:0006217, GO:0006219 Definition: The chemical reactions and pathways resulting in the breakdown of any one of a family of organic molecules consisting of a pyrimidine base covalently bonded to a sugar deoxyribose (a deoxyribonucleoside). Sources: GOC:ai